{
  "gene_symbol": "SLC4A1",
  "term_label": "regulation of intracellular pH",
  "term_id": "GO:0051453",
  "gene": "UniProtKB:P02730",
  "gene_name": "Band 3 anion transport protein"
}